{
  "gene_symbol": "CHPF2",
  "gene_name": "Chondroitin sulfate glucuronyltransferase",
  "term_label": "Unknown cellular component",
  "gene": "UniProtKB:Q9P2E5",
  "term_id": "UNKNOWN:0003"
}